{
  "term_label": "regulation of neurotransmitter secretion",
  "term_id": "GO:0046928",
  "gene_name": "Dysferlin",
  "gene_symbol": "DYSF",
  "gene": "UniProtKB:O75923"
}